{
  "term_id": "GO:0019843",
  "term_label": "rRNA binding",
  "gene_symbol": "EMG1",
  "gene": "UniProtKB:Q92979",
  "gene_name": "Ribosomal RNA small subunit methyltransferase NEP1"
}